{
  "gene": "UniProtKB:Q3KNT9",
  "gene_name": "Sperm-egg fusion protein TMEM95",
  "term_label": "acrosomal membrane",
  "term_id": "GO:0002080",
  "gene_symbol": "TMEM95"
}